{
  "gene_symbol": "FHL5",
  "term_label": "positive regulation of transcription by RNA polymerase II",
  "term_id": "GO:0045944",
  "gene": "UniProtKB:Q5TD97",
  "gene_name": "Four and a half LIM domains protein 5"
}